Cdv-dependent cytokinesis [GO:0061639] (biological process) Definition: A cytokinesis that involves a set of conserved proteins including the Cdv proteins, and results in the formation of two similarly sized and shaped cells. References: PMID:18987308 Sources: GOC:dph Relationships: is a type of cytokinesis [GO:0000910]